{
  "term_id": "GO:0001940",
  "gene_name": "Protein STPG4",
  "gene": "UniProtKB:Q8N801",
  "term_label": "male pronucleus",
  "gene_symbol": "STPG4"
}